{
  "gene_name": "Cadherin-2",
  "gene_symbol": "CDH2",
  "term_id": "GO:0008013",
  "term_label": "beta-catenin binding",
  "gene": "UniProtKB:P19022"
}